{
  "term_label": "olfactory receptor activity",
  "gene_name": "Olfactory receptor 10R2",
  "gene": "UniProtKB:Q8NGX6",
  "term_id": "GO:0004984",
  "gene_symbol": "OR10R2"
}